{
  "term_label": "Unknown cellular component",
  "term_id": "UNKNOWN:0003",
  "gene": "UniProtKB:Q9Y243",
  "gene_name": "RAC-gamma serine_threonine-protein kinase",
  "gene_symbol": "AKT3"
}